{
  "term_label": "cytokine activity",
  "gene_symbol": "TNFSF11",
  "gene_name": "Tumor necrosis factor ligand superfamily member 11",
  "gene": "UniProtKB:O14788",
  "term_id": "GO:0005125"
}